{
  "gene_symbol": "RD3",
  "term_id": "UNKNOWN:0003",
  "term_label": "Unknown cellular component",
  "gene_name": "Protein RD3",
  "gene": "UniProtKB:Q7Z3Z2"
}